{
  "term_label": "endoplasmic reticulum",
  "gene_name": "Protein disulfide-isomerase A6",
  "gene": "UniProtKB:Q15084",
  "term_id": "GO:0005783",
  "gene_symbol": "PDIA6"
}